{
  "term_id": "GO:0014069",
  "gene_name": "Protein shisa-7",
  "term_label": "postsynaptic density",
  "gene": "UniProtKB:A6NL88",
  "gene_symbol": "SHISA7"
}